{
  "term_id": "GO:0015629",
  "term_label": "actin cytoskeleton",
  "gene": "UniProtKB:Q99439",
  "gene_name": "Calponin-2",
  "gene_symbol": "CNN2"
}